{
  "gene_name": "Caspase recruitment domain-containing protein 6",
  "term_id": "UNKNOWN:0002",
  "gene": "UniProtKB:Q9BX69",
  "term_label": "Unknown biological process",
  "gene_symbol": "CARD6"
}